oxidized purine nucleobase lesion DNA N-glycosylase activity [GO:0008534] (molecular function) Also known as: 8-oxoguanine DNA glycosylase activity, DNA glycosylase/AP-lyase activity, DNA glycosylase/beta-lyase activity, bifunctional DNA glycosylase activity, oxidized purine base lesion DNA N-glycosylase activity, 2,6-diamino-4-hydroxy-5(N-methyl)formamidopyrimidine-DNA glycosylase activity, 2,6-diamino-4-hydroxy-5N-formamidopyrimidine-DNA glycosylase activity, DNA glycohydrolase [2,6-diamino-4-hydroxy-5-(N-methyl)formamidopyrimide releasing], DNA-formamidopyrimidine glycosylase activity, Fapy-DNA glycosylase activity, Fpg protein, deoxyribonucleate glycosidase activity, formamidopyrimidine-DNA glycosylase activity, purine-specific oxidized base lesion DNA N-glycosylase activity Note: Consider also annotating to the molecular function term 'DNA-(apurinic or apyrimidinic site) lyase activity ; GO:0003906'. References: PMID:11554296 Sources: GOC:elh Subtypes: 8-oxo-7,8-dihydroguanine DNA N-glycosylase activity [GO:0034039] Relationships: is a type of oxidized base lesion DNA N-glycosylase activity [GO:0000702] Definition: Catalysis of the removal of oxidized purine bases by cleaving the N-C1' glycosidic bond between the oxidized purine and the deoxyribose sugar. The reaction involves the formation of a covalent enzyme-substrate intermediate. Release of the enzyme and free base by a beta-elimination or a beta, gamma-elimination mechanism results in the cleavage of the DNA backbone 3' of the apurinic (AP) site.